positive regulation of cardioblast differentiation [GO:0051891] (biological process) Also known as: up regulation of cardioblast differentiation, up-regulation of cardioblast differentiation, upregulation of cardioblast differentiation, activation of cardioblast differentiation, stimulation of cardioblast differentiation Subtypes: positive regulation of cardiac muscle cell myoblast differentiation [GO:2000700] Sources: GOC:ai Definition: Any process that activates or increases the frequency, rate or extent of cardioblast differentiation, the process in which a relatively unspecialized mesodermal cell acquires the specialized structural and/or functional features of a cardioblast. A cardioblast is a cardiac precursor cell. It is a cell that has been committed to a cardiac fate, but will undergo more cell division rather than terminally differentiating. Relationships: is a type of regulation of cardioblast differentiation [GO:0051890]; is a type of positive regulation of cardiocyte differentiation [GO:1905209]; is a type of positive regulation of stem cell differentiation [GO:2000738]; positively regulates GO:0010002